defense response to insect [GO:0002213] (biological process) Also known as: physiological defense response to insect Definition: A response to protect an organism from a directly detected or perceived external threat from an insect or insects to that organism. Regulation: negatively regulated by negative regulation of defense response to insect [GO:1900366]; positively regulated by positive regulation of defense response to insect [GO:1900367]; regulated by regulation of defense response to insect [GO:2000068] Relationships: is a type of defense response [GO:0006952]; is a type of response to other organism [GO:0051707] Sources: GOC:add Subtypes: behavioral defense response to insect [GO:0002211]